{
  "gene": "UniProtKB:O15273",
  "term_id": "GO:0035995",
  "term_label": "detection of muscle stretch",
  "gene_name": "Telethonin",
  "gene_symbol": "TCAP"
}